{
  "gene_symbol": "POLG2",
  "term_id": "GO:0006264",
  "term_label": "mitochondrial DNA replication",
  "gene": "UniProtKB:Q9UHN1",
  "gene_name": "DNA polymerase subunit gamma-2, mitochondrial"
}